{
  "term_label": "calcium ion binding",
  "gene_name": "Putative inactive group IIC secretory phospholipase A2",
  "term_id": "GO:0005509",
  "gene": "UniProtKB:Q5R387",
  "gene_symbol": "PLA2G2C"
}